establishment of T cell polarity [GO:0001768] (biological process) Also known as: T cell polarization, T lymphocyte polarization, T-cell polarization, establishment of T lymphocyte polarity, establishment of T-cell polarity, establishment of T-lymphocyte polarity Relationships: is a type of establishment of lymphocyte polarity [GO:0001767]; is part of T cell activation [GO:0042110] References: PMID:11244041, PMID:12615889 Sources: GOC:mgi_curators Definition: The directed orientation of T cell signaling molecules and associated membrane rafts towards a chemokine gradient or a contact point with antigen presenting cell. Regulation: regulated by regulation of establishment of T cell polarity [GO:1903903]; RO_0002212 by GO:1903904; positively regulated by GO:1903905